{
  "term_label": "galactose metabolic process",
  "gene_symbol": "GALK1",
  "gene": "UniProtKB:P51570",
  "gene_name": "Galactokinase",
  "term_id": "GO:0006012"
}